negative regulation of DNA damage response, signal transduction by p53 class mediator [GO:0043518] (biological process) Relationships: is a type of GO:0043516; is a type of GO:1901797; negatively regulates DNA damage response, signal transduction by p53 class mediator [GO:0030330] Definition: Any process that stops, prevents, or reduces the frequency, rate or extent of the cascade of processes induced by the cell cycle regulator phosphoprotein p53, or an equivalent protein, in response to the detection of DNA damage. Also known as: down regulation of DNA damage response, signal transduction by p53 class mediator, down-regulation of DNA damage response, signal transduction by p53 class mediator, downregulation of DNA damage response, signal transduction by p53 class mediator, negative regulation of p53 induced by DNA damage response, inhibition of DNA damage response, signal transduction by p53 class mediator Sources: GOC:jl